inner ear receptor cell development [GO:0060119] (BP) Subtypes: auditory receptor cell development [GO:0060117], vestibular receptor cell development [GO:0060118] Relationships: is a type of neuron development [GO:0048666]; is part of inner ear receptor cell differentiation [GO:0060113] Definition: The process whose specific outcome is the progression of an inner ear receptor cell over time, from its formation to the mature structure. Cell development does not include the steps involved in committing a cell to a specific fate. Also known as: inner ear hair cell development Sources: GOC:dph